etioplast [GO:0009513] (cellular component) Definition: A plastid arrested in the development of chloroplasts from proplastids due to absence of light or low light conditions. Sources: ISBN:0943088399 Relationships: is a type of plastid [GO:0009536]